{
  "term_id": "GO:0005109",
  "gene_symbol": "ZNRF3",
  "term_label": "frizzled binding",
  "gene_name": "E3 ubiquitin-protein ligase ZNRF3",
  "gene": "UniProtKB:Q9ULT6"
}